interleukin-6 receptor activity [GO:0004915] (molecular function) Sources: GOC:jl, GOC:signaling Also known as: IL-6 receptor activity, IL-6R, gp130 Relationships: is a type of GO:0004896; is part of interleukin-6-mediated signaling pathway [GO:0070102]; has part interleukin-6 binding [GO:0019981] Definition: Combining with interleukin-6 and transmitting the signal from one side of the membrane to the other to initiate a change in cell activity.